{
  "term_label": "mitotic G2 DNA damage checkpoint signaling",
  "gene": "UniProtKB:Q7Z2Z1",
  "gene_name": "Treslin",
  "gene_symbol": "TICRR",
  "term_id": "GO:0007095"
}